nuclease activity [GO:0004518] (molecular function) Note: Most nucleases are classed as hydrolases, though a minority are classed as lyases. Relationships: is_a GO:0140640 Regulation: negatively regulated by nuclease inhibitor activity [GO:0140721]; positively regulated by GO:0170053 Sources: ISBN:0198547684 Subtypes: endonuclease activity [GO:0004519], exonuclease activity [GO:0004527], DNA nuclease activity [GO:0004536], RNA nuclease activity [GO:0004540] Definition: Catalysis of the cleavage of ester linkages within nucleic acids.